very-low-density lipoprotein particle binding [GO:0034189] (molecular function) Definition: Binding to a very-low-density lipoprotein particle, a triglyceride-rich lipoprotein particle that is typically composed of APOB100, APOE and APOCs and has a density of about 1.006 g/ml and a diameter of between 20-80 nm. Sources: GOC:BHF, GOC:mah Also known as: VLDL binding, very-low-density lipoprotein binding Relationships: is a type of GO:0005515; is a type of lipoprotein particle binding [GO:0071813]